cellular response to nicotine [GO:0071316] (biological process) Definition: Any process that results in a change in state or activity of a cell (in terms of movement, secretion, enzyme production, gene expression, etc.) as a result of a nicotine stimulus. Relationships: is a type of response to nicotine [GO:0035094]; is a type of cellular response to chemical stimulus [GO:0070887] Sources: GOC:mah